{
  "gene": "UniProtKB:Q15700",
  "gene_name": "Disks large homolog 2",
  "term_label": "neuron projection",
  "gene_symbol": "DLG2",
  "term_id": "GO:0043005"
}